{
  "gene_symbol": "PLAGL1",
  "term_id": "GO:0005654",
  "gene_name": "Zinc finger protein PLAGL1",
  "term_label": "nucleoplasm",
  "gene": "UniProtKB:Q9UM63"
}